positive regulation of convergent extension involved in somitogenesis [GO:1904129] (biological process) Definition: Any process that activates or increases the frequency, rate or extent of convergent extension involved in somitogenesis. Relationships: is a type of positive regulation of convergent extension involved in axis elongation [GO:1901234]; is a type of positive regulation of convergent extension involved in gastrulation [GO:1904105]; is a type of GO:1904127; positively regulates convergent extension involved in somitogenesis [GO:0090246] References: PMID:24892953 Sources: GOC:TermGenie, GOC:dph, GO_REF:0000058 Also known as: up regulation of convergent extension involved in somitogenesis, up-regulation of convergent extension involved in somitogenesis, upregulation of convergent extension involved in somitogenesis, activation of convergent extension involved in somitogenesis